keratinocyte apoptotic process [GO:0097283] (biological process) References: PMID:10201527 Sources: CL:0000312, GOC:jc, GOC:mtg_apoptosis Relationships: is a type of GO:1904019 Also known as: keratinocyte apoptosis Regulation: regulated by regulation of keratinocyte apoptotic process [GO:1902172]; negatively regulated by negative regulation of keratinocyte apoptotic process [GO:1902173]; positively regulated by GO:1902174 Definition: Any apoptotic process in a keratinocyte. A keratinocyte is an epidermal cell which synthesizes keratin and undergoes a characteristic change as it moves upward from the basal layers of the epidermis to the cornified (horny) layer of the skin.